{
  "term_id": "GO:0005634",
  "gene_symbol": "ZNF132",
  "gene": "UniProtKB:P52740",
  "gene_name": "Zinc finger protein 132",
  "term_label": "nucleus"
}